sleep [GO:0030431] (biological process) Sources: ISBN:0192800981 Relationships: is a type of GO:0032501 Also known as: diapause, dormancy, lethargus Subtypes: GO:0050802 Definition: Any process in which an organism enters and maintains a periodic, readily reversible state of reduced awareness and metabolic activity. Usually accompanied by physical relaxation, the onset of sleep in humans and other mammals is marked by a change in the electrical activity of the brain.